hydrolase activity, acting on acid anhydrides, in sulfonyl-containing anhydrides [GO:0016819] (molecular function) Definition: Catalysis of the hydrolysis of any acid anhydride which contains a sulfonyl group, -SO2-. Relationships: is a type of hydrolase activity, acting on acid anhydrides [GO:0016817] Also known as: hydrolase activity, acting on acid anhydrides, in sulphonyl-containing anhydrides Sources: GOC:ai Subtypes: GO:0047627, phosphoadenylylsulfatase activity [GO:0050186]